{
  "term_id": "GO:0005886",
  "term_label": "plasma membrane",
  "gene_name": "Interleukin-22 receptor subunit alpha-1",
  "gene_symbol": "IL22RA1",
  "gene": "UniProtKB:Q8N6P7"
}